peptidyl-tyrosine dephosphorylation [GO:0035335] (biological process) Sources: GOC:bf Subtypes: peptidyl-tyrosine dephosphorylation involved in inactivation of protein kinase activity [GO:1990264] Definition: The removal of phosphoric residues from peptidyl-O-phospho-tyrosine to form peptidyl-tyrosine. Relationships: is a type of protein dephosphorylation [GO:0006470]